regulation of long-term neuronal synaptic plasticity [GO:0048169] (biological process) Definition: A process that modulates long-term neuronal synaptic plasticity, the ability of neuronal synapses to change long-term as circumstances require. Long-term neuronal synaptic plasticity generally involves increase or decrease in actual synapse numbers. Subtypes: positive regulation of long-term neuronal synaptic plasticity [GO:0048170], negative regulation of long-term neuronal synaptic plasticity [GO:0048171] Note: Note that the syntax of the definition of this term is different from the usual regulation syntax because it describes regulation of a trait rather than regulation of a process. References: PMID:11891290 Sources: GOC:jid Relationships: is a type of regulation of neuronal synaptic plasticity [GO:0048168]